{
  "gene": "UniProtKB:Q5JTH9",
  "term_label": "nucleolus",
  "term_id": "GO:0005730",
  "gene_name": "RRP12-like protein",
  "gene_symbol": "RRP12"
}